mRNA N1-methyladenosine dioxygenase activity [GO:1990930] (molecular function) References: PMID:26863196, PMID:26863410 Also known as: RNA N(1)-methyladenosine dioxygenase activity, RNA N1-methyladenosine dioxygenase activity Relationships: is a type of oxidative RNA demethylase activity [GO:0035515] Definition: Catalysis of the oxidative demethylation of N1-methyladenosine RNA, with concomitant decarboxylation of 2-oxoglutarate and releases oxidized methyl group on N1-methyladenosine as formaldehyde.